vanillyl-alcohol oxidase activity [GO:0018465] (molecular function) Also known as: 4-hydroxy-2-methoxybenzyl alcohol oxidase activity, vanillyl alcohol:oxygen oxidoreductase activity Relationships: is a type of oxidoreductase activity, acting on the CH-OH group of donors, oxygen as acceptor [GO:0016899] Definition: Catalysis of the reaction: O2 + vanillyl alcohol = H2O2 + vanillin. Sources: EC:1.1.3.38, RHEA:10036